{
  "term_id": "GO:0007015",
  "gene_name": "Coronin-2B",
  "term_label": "actin filament organization",
  "gene": "UniProtKB:Q9UQ03",
  "gene_symbol": "CORO2B"
}